{
  "gene": "UniProtKB:Q9NPE3",
  "term_label": "box H/ACA snoRNP complex",
  "term_id": "GO:0031429",
  "gene_name": "H_ACA ribonucleoprotein complex subunit 3",
  "gene_symbol": "NOP10"
}